{
  "gene_symbol": "SLC45A4",
  "term_label": "Unknown biological process",
  "gene": "UniProtKB:Q5BKX6",
  "gene_name": "Solute carrier family 45 member 4",
  "term_id": "UNKNOWN:0002"
}